{
  "term_label": "endoplasmic reticulum",
  "gene": "UniProtKB:Q53EL9",
  "gene_name": "Seizure protein 6 homolog",
  "term_id": "GO:0005783",
  "gene_symbol": "SEZ6"
}